{
  "gene_symbol": "Q8TAT8",
  "term_id": "UNKNOWN:0001",
  "gene_name": "Putative uncharacterized protein LOC644613",
  "gene": "UniProtKB:Q8TAT8",
  "term_label": "Unknown molecular function"
}